dolichyl-xylosyl-phosphate-protein xylosyltransferase activity [GO:0047284] (molecular function) Definition: Catalysis of the reaction: dolichyl D-xylosyl phosphate + protein = dolichol-phosphate + D-xylosylprotein. Sources: EC:2.4.2.33, MetaCyc:2.4.2.33-RXN Also known as: dolichyl-D-xylosyl-phosphate:protein D-xylosyltransferase activity Relationships: is a type of xylosyltransferase activity [GO:0042285]